symbiont-mediated suppression of host complement activation by activation of host proteases [GO:0141203] (biological process) Also known as: symbiont-mediated suppression of host complement activation by recruitment of host proteases Relationships: is a type of symbiont-mediated suppression of host complement activation [GO:0042784] References: PMID:15792635, PMID:26945067, PMID:34305859 Definition: A process by which a symbiont prevents host complement activation by recruiting host proteases, destroying the complement before it has its effect on the symbiont.